{
  "term_label": "signaling receptor activity",
  "gene_name": "Integrin alpha-V",
  "gene_symbol": "ITGAV",
  "term_id": "GO:0038023",
  "gene": "UniProtKB:P06756"
}